tapasin binding [GO:0046980] (molecular function) Definition: Binding to tapasin, a member of the MHC class I loading complex which bridges the TAP peptide transporter to class I molecules. References: PMID:12594855 Also known as: TAP binding protein binding, TAPBP binding Relationships: is a type of protein binding [GO:0005515]